{
  "term_id": "GO:0050766",
  "gene_name": "High affinity immunoglobulin gamma Fc receptor I",
  "gene_symbol": "FCGR1A",
  "term_label": "positive regulation of phagocytosis",
  "gene": "UniProtKB:P12314"
}